{
  "term_label": "quinol-cytochrome-c reductase activity",
  "term_id": "GO:0008121",
  "gene": "UniProtKB:P00156",
  "gene_symbol": "MT-CYB",
  "gene_name": "Cytochrome b"
}